{
  "term_label": "immune response",
  "gene_symbol": "CD1D",
  "term_id": "GO:0006955",
  "gene_name": "Antigen-presenting glycoprotein CD1d",
  "gene": "UniProtKB:P15813"
}